{
  "gene_name": "Otoraplin",
  "term_id": "GO:0001502",
  "term_label": "cartilage condensation",
  "gene": "UniProtKB:Q9NRC9",
  "gene_symbol": "OTOR"
}